{
  "term_id": "UNKNOWN:0002",
  "gene_symbol": "SMIM10L1",
  "gene": "UniProtKB:P0DMW3",
  "term_label": "Unknown biological process",
  "gene_name": "Small integral membrane protein 10-like protein 1"
}